{
  "term_id": "GO:0019276",
  "gene_name": "Beta-1,4 N-acetylgalactosaminyltransferase 2",
  "gene": "UniProtKB:Q8NHY0",
  "term_label": "UDP-N-acetylgalactosamine metabolic process",
  "gene_symbol": "B4GALNT2"
}